regulation of monocyte aggregation [GO:1900623] (biological process) Subtypes: negative regulation of monocyte aggregation [GO:1900624], positive regulation of monocyte aggregation [GO:1900625] Definition: Any process that modulates the frequency, rate or extent of monocyte aggregation. Relationships: is a type of regulation of leukocyte cell-cell adhesion [GO:1903037]; regulates GO:0070487 Sources: GOC:BHF, GOC:TermGenie Also known as: regulation of mononuclear phagocyte aggregation